{
  "term_id": "UNKNOWN:0002",
  "gene_name": "Neuronal pentraxin receptor",
  "gene_symbol": "NPTXR",
  "gene": "UniProtKB:O95502",
  "term_label": "Unknown biological process"
}